{
  "term_label": "disulfide oxidoreductase activity",
  "gene_symbol": "TMX2",
  "term_id": "GO:0015036",
  "gene": "UniProtKB:Q9Y320",
  "gene_name": "Thioredoxin-related transmembrane protein 2"
}